{
  "gene_symbol": "RPS14",
  "term_id": "GO:0003735",
  "term_label": "structural constituent of ribosome",
  "gene_name": "Small ribosomal subunit protein uS11",
  "gene": "UniProtKB:P62263"
}